positive regulation of inflammatory response to antigenic stimulus [GO:0002863] (biological process) Subtypes: positive regulation of acute inflammatory response to antigenic stimulus [GO:0002866], positive regulation of chronic inflammatory response to antigenic stimulus [GO:0002876] Sources: GOC:add Relationships: is a type of regulation of inflammatory response to antigenic stimulus [GO:0002861]; is a type of positive regulation of inflammatory response [GO:0050729]; is a type of GO:0050778; positively regulates inflammatory response to antigenic stimulus [GO:0002437] Also known as: up regulation of inflammatory response to antigenic stimulus, up-regulation of inflammatory response to antigenic stimulus, upregulation of inflammatory response to antigenic stimulus, activation of inflammatory response to antigenic stimulus, stimulation of inflammatory response to antigenic stimulus Definition: Any process that activates or increases the frequency, rate, or extent of an inflammatory response to an antigenic stimulus.